{
  "gene_symbol": "DUS4L",
  "term_label": "tRNA dihydrouridine synthase activity",
  "gene_name": "tRNA-dihydrouridine(20a_20b) synthase [NAD(P)+]-like",
  "term_id": "GO:0017150",
  "gene": "UniProtKB:O95620"
}